lyso-ornithine lipid acyltransferase activity [GO:0043808] (molecular function) References: PMID:15341653 Definition: Catalysis of the reaction: lyso-ornithine lipid + acyl-[acyl-carrier protein] = ornithine lipid + [acyl-carrier protein]. Relationships: is a type of N-acyltransferase activity [GO:0016410]